{
  "term_id": "GO:0005829",
  "gene_symbol": "WIPI1",
  "term_label": "cytosol",
  "gene_name": "WD repeat domain phosphoinositide-interacting protein 1",
  "gene": "UniProtKB:Q5MNZ9"
}